{
  "gene": "UniProtKB:P20701",
  "gene_symbol": "ITGAL",
  "gene_name": "Integrin alpha-L",
  "term_label": "signaling receptor activity",
  "term_id": "GO:0038023"
}